{
  "gene": "UniProtKB:Q9HCX3",
  "term_id": "GO:0005634",
  "gene_symbol": "ZNF304",
  "gene_name": "Zinc finger protein 304",
  "term_label": "nucleus"
}